{
  "gene_symbol": "NUDT10",
  "gene_name": "Diphosphoinositol polyphosphate phosphohydrolase 3-alpha",
  "gene": "UniProtKB:Q8NFP7",
  "term_label": "bis(5'-adenosyl)-hexaphosphatase activity",
  "term_id": "GO:0034431"
}